{
  "term_id": "GO:0042627",
  "gene": "UniProtKB:P02656",
  "gene_name": "Apolipoprotein C-III",
  "gene_symbol": "APOC3",
  "term_label": "chylomicron"
}